negative regulation of intracellular steroid hormone receptor signaling pathway [GO:0033144] (biological process) Relationships: is_a regulation of intracellular steroid hormone receptor signaling pathway [GO:0033143]; is a type of negative regulation of intracellular signal transduction [GO:1902532]; negatively regulates nuclear receptor-mediated steroid hormone signaling pathway [GO:0030518] Subtypes: negative regulation of intracellular estrogen receptor signaling pathway [GO:0033147], GO:0060766, GO:0120143, GO:2000323 Definition: Any process that stops, prevents, or reduces the frequency, rate or extent of the activity of any intracellular steroid hormone receptor signaling pathway. Also known as: negative regulation of steroid hormone receptor signaling pathway, negative regulation of steroid hormone receptor signalling pathway Sources: GOC:mah